{
  "gene": "UniProtKB:Q07869",
  "gene_name": "Peroxisome proliferator-activated receptor alpha",
  "term_id": "GO:0045923",
  "gene_symbol": "PPARA",
  "term_label": "positive regulation of fatty acid metabolic process"
}